{
  "gene_name": "Glycolipid transfer protein domain-containing protein 2",
  "term_label": "ceramide 1-phosphate transfer activity",
  "gene_symbol": "GLTPD2",
  "term_id": "GO:1902388",
  "gene": "UniProtKB:A6NH11"
}